{
  "term_id": "GO:0007399",
  "gene_name": "UPF0524 protein C3orf70",
  "gene": "UniProtKB:A6NLC5",
  "gene_symbol": "C3orf70",
  "term_label": "nervous system development"
}